{
  "gene_symbol": "GABARAPL3",
  "gene_name": "Gamma-aminobutyric acid receptor-associated protein-like 3",
  "gene": "UniProtKB:Q9BY60",
  "term_id": "GO:0097352",
  "term_label": "autophagosome maturation"
}